{
  "term_label": "olfactory receptor activity",
  "term_id": "GO:0004984",
  "gene": "UniProtKB:Q8NGI0",
  "gene_name": "Olfactory receptor 52N2",
  "gene_symbol": "OR52N2"
}